{
  "gene": "UniProtKB:Q96M86",
  "gene_name": "Dynein heavy chain domain-containing protein 1",
  "term_label": "sperm flagellum",
  "gene_symbol": "DNHD1",
  "term_id": "GO:0036126"
}